xylonate dehydratase activity [GO:0050401] (molecular function) Also known as: D-xylo-aldonate dehydratase activity, D-xylonate dehydratase activity, D-xylonate hydro-lyase (2-dehydro-3-deoxy-D-xylonate-forming), D-xylonate hydro-lyase activity Relationships: is_a hydro-lyase activity [GO:0016836] Definition: Catalysis of the reaction: D-xylonate = 2-dehydro-3-deoxy-D-arabinonate + H2O. Sources: EC:4.2.1.82, RHEA:19157